{
  "gene": "UniProtKB:Q96DS6",
  "gene_name": "Membrane-spanning 4-domains subfamily A member 6E",
  "term_label": "plasma membrane",
  "gene_symbol": "MS4A6E",
  "term_id": "GO:0005886"
}